{
  "term_label": "plasma membrane",
  "term_id": "GO:0005886",
  "gene_symbol": "DRD3",
  "gene_name": "D(3) dopamine receptor",
  "gene": "UniProtKB:P35462"
}